regulation of clathrin-dependent endocytosis [GO:2000369] (biological process) Definition: Any process that modulates the frequency, rate or extent of clathrin-mediated endocytosis. Sources: GOC:mah Also known as: regulation of clathrin coated pit-dependent endocytosis, regulation of clathrin-mediated endocytosis Relationships: is a type of regulation of receptor-mediated endocytosis [GO:0048259]; regulates clathrin-dependent endocytosis [GO:0072583] Subtypes: negative regulation of clathrin-dependent endocytosis [GO:1900186], positive regulation of clathrin-dependent endocytosis [GO:2000370]